{
  "term_label": "Unknown cellular component",
  "gene": "UniProtKB:Q6NUM6",
  "gene_name": "S-adenosyl-L-methionine-dependent tRNA 4-demethylwyosine synthase TYW1B",
  "gene_symbol": "TYW1B",
  "term_id": "UNKNOWN:0003"
}